{
  "term_id": "UNKNOWN:0002",
  "gene_symbol": "MN1",
  "term_label": "Unknown biological process",
  "gene": "UniProtKB:Q10571",
  "gene_name": "Transcriptional activator MN1"
}